{
  "gene_name": "BEN domain-containing protein 5",
  "gene": "UniProtKB:Q7L4P6",
  "term_id": "UNKNOWN:0003",
  "term_label": "Unknown cellular component",
  "gene_symbol": "BEND5"
}